{
  "gene_name": "Rhox homeobox family member 1 pseudogene 3",
  "term_label": "Unknown biological process",
  "gene": "UniProtKB:A0A994J3T1",
  "term_id": "UNKNOWN:0002",
  "gene_symbol": "RHOXF1P3"
}